{
  "term_id": "UNKNOWN:0002",
  "gene_name": "Dual oxidase maturation factor 1",
  "term_label": "Unknown biological process",
  "gene": "UniProtKB:Q1HG43",
  "gene_symbol": "DUOXA1"
}